{
  "gene": "UniProtKB:O15121",
  "gene_symbol": "DEGS1",
  "term_id": "UNKNOWN:0003",
  "gene_name": "Sphingolipid delta(4)-desaturase DES1",
  "term_label": "Unknown cellular component"
}